dorsal closure [GO:0007391] (BP) Definition: The process during Drosophila embryogenesis whereby the ectodermal cells of the lateral epithelium stretch in a coordinated fashion to internalize the amnioserosa cells and close the embryo dorsally. Relationships: is a type of morphogenesis of embryonic epithelium [GO:0016331]; is part of embryonic development via the syncytial blastoderm [GO:0001700] References: PMID:9224720